{
  "gene_symbol": "CBL",
  "term_label": "membrane raft",
  "gene_name": "E3 ubiquitin-protein ligase CBL",
  "gene": "UniProtKB:P22681",
  "term_id": "GO:0045121"
}